galactoside 2-alpha-L-fucosyltransferase activity [GO:0008107] (molecular function) Sources: EC:2.4.1.69, RHEA:50664 Definition: Catalysis of the reaction: GDP-L-fucose + beta-D-galactosyl-R = GDP + alpha-L-fucosyl-(1,2)-beta-D-galactosyl-R. Relationships: is a type of GO:0031127 Also known as: alpha(1,2)-L-fucosyltransferase activity, H-gene-encoded beta-galactoside alpha-1->2 fucosyltransferase activity, blood group H alpha-2-fucosyltransferase activity, blood-group substance H-dependent fucosyltransferase activity, secretor-type beta-galactoside alpha-1->2 fucosyltransferase activity, GDP fucose-lactose fucosyltransferase activity, GDP-L-fucose:lactose fucosyltransferase activity, GDP-beta-L-fucose:beta-D-galactosyl-R 2-alpha-L-fucosyltransferase activity, H-gene-encoded beta-galactoside alpha1->2 fucosyltransferase activity, alpha-(1->2)-L-fucosyltransferase activity, alpha-2-L-fucosyltransferase activity, alpha-2-fucosyltransferase activity, beta-galactoside alpha-1->2 fucosyltransferase activity, beta-galactoside alpha1->2 fucosyltransferase activity, galactoside 2-L-fucosyltransferase activity, guanosine diphospho-L-fucose-lactose fucosyltransferase activity, guanosine diphosphofucose-beta-D-galactosyl-alpha-2-L-fucosyltransferase activity, guanosine diphosphofucose-galactoside 2-L-fucosyltransferase activity, guanosine diphosphofucose-galactosylacetylglucosaminylgalactosyl-glucosylceramide alpha-L-fucosyltransferase activity, guanosine diphosphofucose-galactosylacetylglucosaminylgalactosylglucosylceramide alpha-L-fucosyltransferase activity, guanosine diphosphofucose-glycoprotein 2-alpha-L-fucosyltransferase activity, guanosine diphosphofucose-glycoprotein 2-alpha-fucosyltransferase activity, guanosine diphosphofucose-lactose fucosyltransferase activity, secretor-type beta-galactoside alpha1->2 fucosyltransferase activity